{
  "gene": "UniProtKB:O15062",
  "gene_symbol": "ZBTB5",
  "term_id": "GO:0006357",
  "gene_name": "Zinc finger and BTB domain-containing protein 5",
  "term_label": "regulation of transcription by RNA polymerase II"
}